{
  "term_label": "heterophilic cell-cell adhesion",
  "gene_symbol": "CEACAM19",
  "gene_name": "Carcinoembryonic antigen-related cell adhesion molecule 19",
  "term_id": "GO:0007157",
  "gene": "UniProtKB:Q7Z692"
}